{
  "term_label": "piRNA processing",
  "gene_symbol": "PIWIL3",
  "gene": "UniProtKB:Q7Z3Z3",
  "gene_name": "Piwi-like protein 3",
  "term_id": "GO:0034587"
}